{
  "term_label": "hydroxymethylglutaryl-CoA synthase activity",
  "term_id": "GO:0004421",
  "gene_name": "Hydroxymethylglutaryl-CoA synthase, cytoplasmic",
  "gene_symbol": "HMGCS1",
  "gene": "UniProtKB:Q01581"
}